{
  "term_label": "DNA-binding transcription factor activity, RNA polymerase II-specific",
  "gene_symbol": "ZFP69",
  "term_id": "GO:0000981",
  "gene": "UniProtKB:Q49AA0",
  "gene_name": "Zinc finger protein 69 homolog"
}